phosphoribosylanthranilate isomerase activity [GO:0004640] (molecular function) Relationships: is a type of intramolecular oxidoreductase activity, interconverting aldoses and ketoses [GO:0016861] Also known as: IGPS:PRAI (indole-3-glycerol-phosphate synthetase/N-5'-phosphoribosylanthranilate isomerase complex), N-(5'-phosphoribosyl)anthranilate isomerase activity, N-(5-phospho-beta-D-ribosyl)anthranilate aldose-ketose-isomerase activity, N-(5-phospho-beta-D-ribosyl)anthranilate ketol-isomerase activity, PRA isomerase activity, PRAI activity Definition: Catalysis of the reaction: N-(5-phospho-beta-D-ribosyl)anthranilate = 1-(2-carboxyphenylamino)-1-deoxy-D-ribulose 5-phosphate. Sources: RHEA:21540